{
  "gene": "UniProtKB:P23276",
  "gene_name": "Kell blood group glycoprotein",
  "gene_symbol": "KEL",
  "term_id": "GO:0005886",
  "term_label": "plasma membrane"
}